{
  "gene_name": "Metal transporter CNNM4",
  "gene_symbol": "CNNM4",
  "term_id": "GO:0005886",
  "gene": "UniProtKB:Q6P4Q7",
  "term_label": "plasma membrane"
}